{
  "term_label": "Unknown molecular function",
  "term_id": "UNKNOWN:0001",
  "gene": "UniProtKB:Q9Y5M8",
  "gene_name": "Signal recognition particle receptor subunit beta",
  "gene_symbol": "SRPRB"
}